spindle elongation [GO:0051231] (biological process) Sources: GOC:ai Regulation: regulated by GO:0032887 Relationships: is a type of GO:0007017; is a type of GO:0022402; is part of GO:0007051; is part of nuclear chromosome segregation [GO:0098813] Definition: The cell cycle process in which the distance is lengthened between poles of the spindle. Subtypes: mitotic spindle elongation [GO:0000022], GO:0051232